metanephric loop of Henle development [GO:0072236] (biological process) Relationships: is a type of loop of Henle development [GO:0072070]; is a type of metanephric nephron tubule development [GO:0072234] Also known as: metanephric intermediate tubule development Definition: The process whose specific outcome is the progression of the metanephric loop of Henle over time, from its formation to the mature structure. The metanephric loop of Henle is a metanephric nephron tubule that connects the proximal convoluted tubule to the distal convoluted tubule in the metanephros. Sources: GOC:mtg_kidney_jan10